{
  "gene": "UniProtKB:Q8IWW8",
  "gene_name": "Hydroxyacid-oxoacid transhydrogenase, mitochondrial",
  "term_label": "alcohol dehydrogenase (NAD+) activity",
  "gene_symbol": "ADHFE1",
  "term_id": "GO:0004022"
}